{
  "gene_symbol": "SLC4A3",
  "gene": "UniProtKB:P48751",
  "term_id": "GO:0055085",
  "term_label": "transmembrane transport",
  "gene_name": "Anion exchange protein 3"
}